{
  "gene": "UniProtKB:Q9BWF2",
  "gene_name": "E3 ubiquitin-protein ligase TRAIP",
  "term_id": "GO:0005634",
  "gene_symbol": "TRAIP",
  "term_label": "nucleus"
}